stress-activated MAPK cascade [GO:0051403] (biological process) Relationships: is_a MAPK cascade [GO:0000165]; is a type of stress-activated protein kinase signaling cascade [GO:0031098] Also known as: SAPK cascade, stress-activated MAPK signaling pathway, stress-activated MAPK signalling pathway, stress-activated MAPKKK cascade, stress-activated MAPKKK signaling pathway, stress-activated MAPKKK signalling pathway, MAPK11 cascade, MAPK12 cascade, MAPK13 cascade, MAPK14 cascade References: PMID:15936270 Sources: GOC:ai Regulation: regulated by GO:0032872; negatively regulated by negative regulation of stress-activated MAPK cascade [GO:0032873]; positively regulated by GO:0032874 Subtypes: cell integrity MAPK cascade [GO:0000196], filamentous growth MAPK cascade [GO:0062031] Definition: A MAPK cascade that starts with the activation of a stress-activated MAP kinase cascade.